{
  "gene": "UniProtKB:P0C869",
  "gene_symbol": "PLA2G4B",
  "gene_name": "Cytosolic phospholipase A2 beta",
  "term_id": "GO:0046475",
  "term_label": "glycerophospholipid catabolic process"
}